regulation of protein folding [GO:1903332] (biological process) Definition: Any process that modulates the frequency, rate or extent of protein folding. Sources: GOC:TermGenie, GOC:vw, GO_REF:0000058 Relationships: is a type of regulation of cellular process [GO:0050794]; regulates protein folding [GO:0006457] Also known as: regulation of alpha-tubulin folding, regulation of beta-tubulin folding, regulation of chaperonin-mediated tubulin folding, regulation of chaperone activity, regulation of chaperonin ATPase activity, regulation of co-chaperone activity, regulation of co-chaperonin activity, regulation of glycoprotein-specific chaperone activity, regulation of non-chaperonin molecular chaperone ATPase activity, regulation of protein complex assembly, multichaperone pathway Subtypes: regulation of protein folding in endoplasmic reticulum [GO:0060904], regulation of protein refolding [GO:0061083], negative regulation of protein folding [GO:1903333], positive regulation of protein folding [GO:1903334]